{
  "gene": "UniProtKB:Q86VI3",
  "term_label": "cell cortex",
  "gene_symbol": "IQGAP3",
  "term_id": "GO:0005938",
  "gene_name": "Ras GTPase-activating-like protein IQGAP3"
}